{
  "gene": "UniProtKB:Q8NGC6",
  "term_id": "UNKNOWN:0003",
  "gene_symbol": "OR4K17",
  "term_label": "Unknown cellular component",
  "gene_name": "Olfactory receptor 4K17"
}